{
  "gene_name": "Kanadaptin",
  "gene_symbol": "SLC4A1AP",
  "term_label": "Unknown cellular component",
  "term_id": "UNKNOWN:0003",
  "gene": "UniProtKB:Q9BWU0"
}